{
  "gene_name": "A-kinase anchor protein 10, mitochondrial",
  "gene": "UniProtKB:O43572",
  "term_label": "plasma membrane",
  "term_id": "GO:0005886",
  "gene_symbol": "AKAP10"
}